{
  "gene_symbol": "PPIF",
  "term_id": "GO:0016018",
  "gene_name": "Peptidyl-prolyl cis-trans isomerase F, mitochondrial",
  "gene": "UniProtKB:P30405",
  "term_label": "cyclosporin A binding"
}